{
  "term_label": "mitochondrion",
  "gene_symbol": "PAAT",
  "term_id": "GO:0005739",
  "gene": "UniProtKB:Q9H8K7",
  "gene_name": "ATPase PAAT"
}